{
  "gene": "UniProtKB:Q9BSJ8",
  "term_id": "GO:0005509",
  "gene_name": "Extended synaptotagmin-1",
  "gene_symbol": "ESYT1",
  "term_label": "calcium ion binding"
}